{
  "gene": "UniProtKB:Q9H251",
  "term_label": "beta-catenin binding",
  "term_id": "GO:0008013",
  "gene_symbol": "CDH23",
  "gene_name": "Cadherin-23"
}